methylglyoxal reductase (NADPH) activity [GO:0043892] (molecular function) Also known as: lactaldehyde dehydrogenase (NADP+), methylglyoxal reductase (NADPH-dependent) activity, Gre2, lactaldehyde:NADP+ oxidoreductase activity Definition: Catalysis of the reaction: lactaldehyde + NADP+ = methylglyoxal + NADPH + H+. Relationships: is a type of GO:0016616 Sources: EC:1.1.1.283